{
  "term_id": "GO:0004984",
  "term_label": "olfactory receptor activity",
  "gene": "UniProtKB:Q9H209",
  "gene_name": "Olfactory receptor 10A4",
  "gene_symbol": "OR10A4"
}